{
  "gene_name": "Protein shisa-9",
  "term_label": "dendritic spine membrane",
  "gene": "UniProtKB:B4DS77",
  "term_id": "GO:0032591",
  "gene_symbol": "SHISA9"
}